{
  "term_label": "extracellular space",
  "gene_name": "Antigen-presenting glycoprotein CD1d",
  "term_id": "GO:0005615",
  "gene_symbol": "CD1D",
  "gene": "UniProtKB:P15813"
}